{
  "gene_symbol": "ACSL5",
  "term_id": "GO:0005783",
  "term_label": "endoplasmic reticulum",
  "gene": "UniProtKB:Q9ULC5",
  "gene_name": "Long-chain-fatty-acid--CoA ligase 5"
}